ATPase-coupled polar amino acid-transporter activity [GO:0015426] (molecular function) Definition: Enables the transfer of a solute or solutes from one side of a membrane to the other according to the reaction: ATP + H2O + polar amino acid(out) = ADP + phosphate + polar amino acid(in). Sources: EC:7.4.2.1 Also known as: ATP-dependent polar amino acid-transporter activity, polar amino acid uptake transporter activity, polar amino acid-importing ATPase activity, polar-amino acid-importing ATPase activity, polar-amino acid-transporting ATPase activity, histidine permease activity, polar-amino acid ABC transporter, cystine/diaminopimelate porter activity, glutamate/aspartate porter activity, histidine/arginine/lysine/ornithine porter activity, polar-amino-acid-transporting ATPase activity Relationships: is a type of GO:0015424 Subtypes: ATPase-coupled L-glutamine transmembrane transporter activity [GO:0015599], GO:0102013